{
  "gene_name": "GRB10-interacting GYF protein 2",
  "term_label": "insulin-like growth factor receptor signaling pathway",
  "gene": "UniProtKB:Q6Y7W6",
  "gene_symbol": "GIGYF2",
  "term_id": "GO:0048009"
}